cranial ganglion maturation [GO:0061558] (biological process) Also known as: cranial ganglia maturation Definition: A developmental process, independent of morphogenetic (shape) change, that is required for a cranial ganglion to attain its fully functional state. Relationships: is a type of ganglion maturation [GO:0061553]; is part of cranial nerve maturation [GO:0021605]; is part of cranial ganglion development [GO:0061550] Subtypes: trigeminal ganglion maturation [GO:0061557] Sources: GOC:dph